{
  "gene_name": "Glypican-4",
  "gene": "UniProtKB:O75487",
  "term_id": "GO:0031012",
  "term_label": "extracellular matrix",
  "gene_symbol": "GPC4"
}